{
  "gene_symbol": "FBXL20",
  "gene_name": "F-box_LRR-repeat protein 20",
  "gene": "UniProtKB:Q96IG2",
  "term_id": "UNKNOWN:0001",
  "term_label": "Unknown molecular function"
}